{
  "gene": "UniProtKB:Q9GZS9",
  "gene_name": "Carbohydrate sulfotransferase 5",
  "term_id": "GO:0005802",
  "gene_symbol": "CHST5",
  "term_label": "trans-Golgi network"
}